{
  "gene_name": "Shiftless antiviral inhibitor of ribosomal frameshifting protein",
  "gene": "UniProtKB:Q9NUL5",
  "term_id": "GO:0043022",
  "term_label": "ribosome binding",
  "gene_symbol": "SHFL"
}